{
  "term_label": "Unknown molecular function",
  "gene": "UniProtKB:Q9GIP4",
  "term_id": "UNKNOWN:0001",
  "gene_name": "Putative L-type amino acid transporter 1-like protein IMAA",
  "gene_symbol": "SLC7A5P2"
}